{
  "gene_symbol": "TUBA4A",
  "gene_name": "Tubulin alpha-4A chain",
  "gene": "UniProtKB:P68366",
  "term_id": "GO:0005200",
  "term_label": "structural constituent of cytoskeleton"
}